positive regulation of paraxial mesodermal cell fate specification [GO:0048350] (biological process) Also known as: up regulation of paraxial mesodermal cell fate specification, up-regulation of paraxial mesodermal cell fate specification, upregulation of paraxial mesodermal cell fate specification, activation of paraxial mesodermal cell fate specification, stimulation of paraxial mesodermal cell fate specification Relationships: is_a GO:0048337; is a type of regulation of paraxial mesodermal cell fate specification [GO:0048349]; positively regulates paraxial mesodermal cell fate specification [GO:0048348] Sources: GOC:dgh Definition: Any process that activates or increases the frequency, rate or extent of paraxial mesoderm cell fate specification.